{
  "term_id": "GO:0005184",
  "gene": "UniProtKB:Q5JQD4",
  "gene_symbol": "PYY3",
  "gene_name": "Putative peptide YY-3",
  "term_label": "neuropeptide hormone activity"
}